{
  "term_label": "regulation of transcription by RNA polymerase II",
  "gene_name": "Homeobox protein Hox-B13",
  "gene_symbol": "HOXB13",
  "term_id": "GO:0006357",
  "gene": "UniProtKB:Q92826"
}